{
  "gene_symbol": "AQP3",
  "term_label": "water transport",
  "gene": "UniProtKB:Q92482",
  "gene_name": "Aquaporin-3",
  "term_id": "GO:0006833"
}